positive regulation of coagulation [GO:0050820] (biological process) Also known as: positive regulation of clotting, up regulation of coagulation, up-regulation of coagulation, upregulation of coagulation, activation of coagulation, stimulation of coagulation Sources: GOC:ai Definition: Any process that activates or increases the frequency, rate or extent of coagulation. Subtypes: positive regulation of blood coagulation [GO:0030194] Relationships: is a type of regulation of coagulation [GO:0050818]; is a type of positive regulation of multicellular organismal process [GO:0051240]; positively regulates coagulation [GO:0050817]